{
  "gene_symbol": "ZNF417",
  "term_label": "RNA polymerase II cis-regulatory region sequence-specific DNA binding",
  "gene_name": "Zinc finger protein 417",
  "term_id": "GO:0000978",
  "gene": "UniProtKB:Q8TAU3"
}